{
  "term_label": "regulation of DNA-templated transcription elongation",
  "gene_name": "DBIRD complex subunit ZNF326",
  "gene": "UniProtKB:Q5BKZ1",
  "gene_symbol": "ZNF326",
  "term_id": "GO:0032784"
}